{
  "gene": "UniProtKB:Q6NW34",
  "gene_symbol": "NEPRO",
  "gene_name": "Nucleolus and neural progenitor protein",
  "term_id": "GO:0005634",
  "term_label": "nucleus"
}